{
  "gene_symbol": "CRAT",
  "gene_name": "Carnitine O-acetyltransferase",
  "gene": "UniProtKB:P43155",
  "term_id": "GO:0004092",
  "term_label": "carnitine O-acetyltransferase activity"
}